{
  "gene_name": "Peripheral-type benzodiazepine receptor-associated protein 1",
  "gene": "UniProtKB:O95153",
  "term_label": "mitochondrion",
  "term_id": "GO:0005739",
  "gene_symbol": "TSPOAP1"
}